Dbf4-dependent protein kinase complex [GO:0031431] (cellular component) Also known as: DDK, Cdc7-Dbf4 complex, Hsk1-Dfp1 kinase complex References: PMID:12045100 Definition: A heterodimeric protein complex required for the activation of DNA replication origins; comprises a catalytic subunit and a regulatory subunit (in Saccharomyces, Cdc7p and Dbf4p, respectively); complexes identified in other species generally contain proteins related to the Saccharomyces proteins. Relationships: is a type of nuclear protein-containing complex [GO:0140513]; is a type of serine/threonine protein kinase complex [GO:1902554]